negative regulation of phagocytosis [GO:0050765] (biological process) Also known as: down regulation of phagocytosis, down-regulation of phagocytosis, downregulation of phagocytosis, inhibition of phagocytosis Definition: Any process that stops, prevents, or reduces the frequency, rate or extent of phagocytosis. Relationships: is a type of negative regulation of endocytosis [GO:0045806]; is a type of regulation of phagocytosis [GO:0050764]; negatively regulates phagocytosis [GO:0006909] Sources: GOC:ai Subtypes: GO:0060101, negative regulation of Fc-gamma receptor signaling pathway involved in phagocytosis [GO:1905450], negative regulation of apoptotic cell clearance [GO:2000426]